{
  "term_label": "cytoplasm",
  "gene": "UniProtKB:P22061",
  "gene_symbol": "PCMT1",
  "gene_name": "Protein-L-isoaspartate(D-aspartate) O-methyltransferase",
  "term_id": "GO:0005737"
}